{
  "term_label": "nuclear receptor activity",
  "term_id": "GO:0004879",
  "gene": "UniProtKB:P10826",
  "gene_symbol": "RARB",
  "gene_name": "Retinoic acid receptor beta"
}